{
  "gene": "UniProtKB:Q07075",
  "gene_symbol": "ENPEP",
  "gene_name": "Glutamyl aminopeptidase",
  "term_id": "GO:0043171",
  "term_label": "peptide catabolic process"
}